{
  "term_id": "UNKNOWN:0001",
  "gene": "UniProtKB:P15941",
  "gene_symbol": "MUC1",
  "gene_name": "Mucin-1",
  "term_label": "Unknown molecular function"
}